{
  "term_label": "positive regulation of T cell activation",
  "gene_name": "HLA class II histocompatibility antigen, DO alpha chain",
  "gene_symbol": "HLA-DOA",
  "gene": "UniProtKB:P06340",
  "term_id": "GO:0050870"
}